{
  "gene_symbol": "ZNF880",
  "term_id": "GO:0000981",
  "term_label": "DNA-binding transcription factor activity, RNA polymerase II-specific",
  "gene_name": "Zinc finger protein 880",
  "gene": "UniProtKB:Q6PDB4"
}